{
  "term_id": "GO:1990573",
  "gene": "UniProtKB:Q15842",
  "term_label": "potassium ion import across plasma membrane",
  "gene_symbol": "KCNJ8",
  "gene_name": "ATP-sensitive inward rectifier potassium channel 8"
}